tRNA-dihydrouridine20a synthase activity [GO:0102266] (molecular function) Relationships: is_a tRNA dihydrouridine synthase activity [GO:0017150] Sources: GOC:pz Definition: Catalysis of the reaction: a 5,6-dihydrouracil20a in tRNA + NAD(P) = H+ + a uracil20a in tRNA + NAD(P)H.